{
  "gene": "UniProtKB:Q15436",
  "gene_name": "Protein transport protein Sec23A",
  "term_label": "COPII vesicle coat",
  "term_id": "GO:0030127",
  "gene_symbol": "SEC23A"
}